{
  "term_id": "GO:0001525",
  "gene_name": "Serine_threonine-protein kinase receptor R3",
  "gene": "UniProtKB:P37023",
  "term_label": "angiogenesis",
  "gene_symbol": "ACVRL1"
}